{
  "term_label": "GTPase activity",
  "gene_name": "GTP-binding protein SAR1b",
  "gene_symbol": "SAR1B",
  "term_id": "GO:0003924",
  "gene": "UniProtKB:Q9Y6B6"
}